monoamine transmembrane transporter activity [GO:0008504] (molecular function) Relationships: is a type of GO:0022804; is part of monoamine transport [GO:0015844] Definition: Enables the transfer of monoamines, organic compounds that contain one amino group that is connected to an aromatic ring by an ethylene group (-CH2-CH2-), from one side of a membrane to the other. Sources: GOC:mah Subtypes: dopamine:sodium symporter activity [GO:0005330], GO:0005334, serotonin:sodium:chloride symporter activity [GO:0005335], monoamine:proton antiporter activity [GO:0015311], tyrosine:tyramine antiporter activity [GO:0070908]